{
  "term_label": "cholesterol efflux",
  "term_id": "GO:0033344",
  "gene_name": "Apolipoprotein E",
  "gene_symbol": "APOE",
  "gene": "UniProtKB:P02649"
}